{
  "gene_symbol": "ZNF840P",
  "gene_name": "Putative zinc finger protein 840",
  "gene": "UniProtKB:A6NDX5",
  "term_label": "transcription cis-regulatory region binding",
  "term_id": "GO:0000976"
}